{
  "gene": "UniProtKB:P12429",
  "term_id": "GO:0005634",
  "gene_symbol": "ANXA3",
  "term_label": "nucleus",
  "gene_name": "Annexin A3"
}